{
  "gene": "UniProtKB:A0A0A0MTA7",
  "term_id": "UNKNOWN:0003",
  "gene_symbol": "TRBJ2-1",
  "gene_name": "T cell receptor beta joining 2-1",
  "term_label": "Unknown cellular component"
}